{
  "gene_name": "Beta-defensin 116",
  "gene": "UniProtKB:Q30KQ4",
  "term_label": "Unknown molecular function",
  "gene_symbol": "DEFB116",
  "term_id": "UNKNOWN:0001"
}